{
  "term_id": "GO:0061630",
  "gene_name": "Neuralized-like protein 4",
  "gene_symbol": "NEURL4",
  "term_label": "ubiquitin protein ligase activity",
  "gene": "UniProtKB:Q96JN8"
}